{
  "term_id": "GO:0042742",
  "gene_symbol": "FCER1G",
  "term_label": "defense response to bacterium",
  "gene_name": "High affinity immunoglobulin epsilon receptor subunit gamma",
  "gene": "UniProtKB:P30273"
}